endonuclease activity [GO:0004519] (MF) Sources: GOC:mah, ISBN:0198547684 Relationships: is a type of nuclease activity [GO:0004518] Subtypes: DNA endonuclease activity [GO:0004520], RNA endonuclease activity [GO:0004521] Definition: Catalysis of the cleavage of ester linkages within nucleic acids by creating internal breaks.